{
  "term_label": "negative regulation of BMP signaling pathway",
  "gene": "UniProtKB:Q9HCE7",
  "gene_symbol": "SMURF1",
  "gene_name": "E3 ubiquitin-protein ligase SMURF1",
  "term_id": "GO:0030514"
}